fastigial nucleus development [GO:0021738] (biological process) Sources: GOC:cls, GOC:curators, GOC:dgh, GOC:dph, GOC:jid Relationships: is a type of GO:0048857; is part of GO:0021549 Definition: The process whose specific outcome is the progression of the fastigial nucleus over time, from its formation to the mature structure.